oocyte microtubule cytoskeleton polarization [GO:0008103] (BP) Relationships: is a type of microtubule-based process [GO:0007017]; is part of oocyte axis specification [GO:0007309]; is part of GO:0016325 References: PMID:11807042 Sources: GOC:mtg_sensu Definition: Establishment and maintenance of a specific axis of polarity of the oocyte microtubule network. The axis is set so that the minus and plus ends of the microtubules of the mid stage oocyte are positioned along the anterior cortex and at the posterior pole, respectively. An example of this is found in Drosophila melanogaster.